{
  "gene_name": "Endosomal_lysosomal proton channel TMEM175",
  "gene": "UniProtKB:Q9BSA9",
  "gene_symbol": "TMEM175",
  "term_label": "endosome",
  "term_id": "GO:0005768"
}